regulation of adenylate cyclase-activating G protein-coupled receptor signaling pathway [GO:0106070] (biological process) References: PMID:19246489 Sources: GOC:hjd Subtypes: GO:0106071, negative regulation of adenylate cyclase-activating G protein-coupled receptor signaling pathway [GO:0106072], GO:0110033 Also known as: regulation of adenylate cyclase-activating G-protein coupled receptor signaling pathway Relationships: is a type of GO:0008277; RO_0002211 adenylate cyclase-activating G protein-coupled receptor signaling pathway [GO:0007189] Definition: Any process that modulates the frequency, rate or extent of an adenylate cyclase-activating G protein-coupled receptor signaling pathway.